{
  "gene_symbol": "HDAC2",
  "term_label": "heterochromatin formation",
  "gene_name": "Histone deacetylase 2",
  "gene": "UniProtKB:Q92769",
  "term_id": "GO:0031507"
}